{
  "gene_name": "Olfactory receptor 4F5",
  "term_label": "olfactory receptor activity",
  "term_id": "GO:0004984",
  "gene": "UniProtKB:Q8NH21",
  "gene_symbol": "OR4F5"
}